{
  "gene_symbol": "YJU2",
  "term_label": "mRNA cis splicing, via spliceosome",
  "gene_name": "Splicing factor YJU2",
  "gene": "UniProtKB:Q9BW85",
  "term_id": "GO:0045292"
}